negative regulation of protein K63-linked ubiquitination [GO:1900045] (biological process) Relationships: is a type of regulation of protein K63-linked ubiquitination [GO:1900044]; is a type of negative regulation of protein polyubiquitination [GO:1902915]; negatively regulates protein K63-linked ubiquitination [GO:0070534] Also known as: down regulation of protein K63-linked polyubiquitination, down-regulation of protein K63-linked polyubiquitination, downregulation of protein K63-linked polyubiquitination, inhibition of protein K63-linked polyubiquitination, negative regulation of protein K63-linked polyubiquitination, down regulation of protein K63-linked ubiquitination, down-regulation of protein K63-linked ubiquitination, downregulation of protein K63-linked ubiquitination, inhibition of protein K63-linked ubiquitination Definition: Any process that stops, prevents or reduces the frequency, rate or extent of protein K63-linked ubiquitination. Sources: GOC:TermGenie